{
  "gene": "UniProtKB:Q9Y6E0",
  "gene_symbol": "STK24",
  "gene_name": "Serine_threonine-protein kinase 24",
  "term_label": "Golgi apparatus",
  "term_id": "GO:0005794"
}